{
  "term_label": "plasma membrane",
  "gene_symbol": "DRD5",
  "gene_name": "D(1B) dopamine receptor",
  "term_id": "GO:0005886",
  "gene": "UniProtKB:P21918"
}